negative regulation of coenzyme F420-dependent bicyclic nitroimidazole catabolic process [GO:1900289] (biological process) Relationships: is a type of GO:0009895; is a type of regulation of coenzyme F420-dependent bicyclic nitroimidazole catabolic process [GO:1900288]; negatively regulates coenzyme F420-dependent bicyclic nitroimidazole catabolic process [GO:0052799] Also known as: down regulation of coenzyme F420-dependent bicyclic nitroimidazole catabolic process, down regulation of coenzyme F420-dependent nitroimidazole breakdown, down regulation of coenzyme F420-dependent nitroimidazole catabolism, down regulation of coenzyme F420-dependent nitroimidazole reduction, down-regulation of coenzyme F420-dependent bicyclic nitroimidazole catabolic process, down-regulation of coenzyme F420-dependent nitroimidazole breakdown, down-regulation of coenzyme F420-dependent nitroimidazole catabolism, down-regulation of coenzyme F420-dependent nitroimidazole reduction, downregulation of coenzyme F420-dependent bicyclic nitroimidazole catabolic process, downregulation of coenzyme F420-dependent nitroimidazole breakdown, downregulation of coenzyme F420-dependent nitroimidazole catabolism, downregulation of coenzyme F420-dependent nitroimidazole reduction, negative regulation of coenzyme F420-dependent nitroimidazole breakdown, negative regulation of coenzyme F420-dependent nitroimidazole catabolism, negative regulation of coenzyme F420-dependent nitroimidazole reduction, inhibition of coenzyme F420-dependent bicyclic nitroimidazole catabolic process, inhibition of coenzyme F420-dependent nitroimidazole breakdown, inhibition of coenzyme F420-dependent nitroimidazole catabolism, inhibition of coenzyme F420-dependent nitroimidazole reduction, down regulation of coenzyme F420-dependent nitroreductase activity, down-regulation of coenzyme F420-dependent nitroreductase activity, downregulation of coenzyme F420-dependent nitroreductase activity, inhibition of coenzyme F420-dependent nitroreductase activity, negative regulation of coenzyme F420-dependent nitroreductase activity Definition: Any process that stops, prevents or reduces the frequency, rate or extent of coenzyme F420-dependent bicyclic nitroimidazole catabolic process. Sources: GOC:TermGenie, GOC:mengo_curators